{
  "gene": "UniProtKB:P02545",
  "term_label": "protein localization to nuclear envelope",
  "gene_symbol": "LMNA",
  "gene_name": "Prelamin-A_C",
  "term_id": "GO:0090435"
}